{
  "term_id": "GO:0005634",
  "term_label": "nucleus",
  "gene": "UniProtKB:P78413",
  "gene_name": "Iroquois-class homeodomain protein IRX-4",
  "gene_symbol": "IRX4"
}